{
  "gene_symbol": "SPEF2",
  "gene": "UniProtKB:Q9C093",
  "gene_name": "Sperm flagellar protein 2",
  "term_label": "Unknown molecular function",
  "term_id": "UNKNOWN:0001"
}